negative regulation of nitric-oxide synthase activity [GO:0051001] (biological process) Sources: GOC:ai Definition: Any process that stops or reduces the activity of the enzyme nitric-oxide synthase. Also known as: down regulation of nitric-oxide synthase activity, down-regulation of nitric-oxide synthase activity, downregulation of nitric-oxide synthase activity, negative regulation of NOS activity, NOS inhibitor, inhibition of nitric-oxide synthase activity, nitric-oxide synthase inhibitor Relationships: is_a regulation of nitric-oxide synthase activity [GO:0050999]; is a type of negative regulation of oxidoreductase activity [GO:0051354]; negatively regulates nitric-oxide synthase activity [GO:0004517]